{
  "term_label": "Cul2-RING ubiquitin ligase complex",
  "gene": "UniProtKB:A3QJZ6",
  "term_id": "GO:0031462",
  "gene_symbol": "PRAMEF22",
  "gene_name": "PRAME family member 22"
}